{
  "gene_name": "MAP_microtubule affinity-regulating kinase 3",
  "gene": "UniProtKB:P27448",
  "term_id": "GO:0005737",
  "term_label": "cytoplasm",
  "gene_symbol": "MARK3"
}